{
  "gene_name": "Interleukin-15",
  "term_id": "GO:0050778",
  "term_label": "positive regulation of immune response",
  "gene_symbol": "IL15",
  "gene": "UniProtKB:P40933"
}